{
  "term_id": "GO:0042721",
  "gene_symbol": "TIMM22",
  "gene": "UniProtKB:Q9Y584",
  "term_label": "TIM22 mitochondrial import inner membrane insertion complex",
  "gene_name": "Mitochondrial import inner membrane translocase subunit Tim22"
}